synaptobrevin 2-SNAP-25-syntaxin-3-complexin complex [GO:0070554] (cellular component) References: PMID:8824312 Relationships: is a type of SNARE complex [GO:0031201] Also known as: SNARE complex (Stx3, Snap25, Vamp2, Cplx1), Stx3-Snap25-Vamp2-Cplx1 complex Definition: A SNARE complex that contains synaptobrevin 2 (VAMP2), SNAP-25, syntaxin 3, and a complexin (or orthologs thereof).